pectin acetylesterase activity [GO:0052793] (molecular function) Definition: Catalysis of the reaction: pectin + H2O = pectate + acetate. This reaction is the hydrolysis of acetyl esters of pectin, producing pectate, partially esterified pectin. Relationships: is a type of carboxylic ester hydrolase activity [GO:0052689] References: PMID:9218776 Sources: GOC:mengo_curators